{
  "term_label": "cytoplasm",
  "gene_name": "Melanocortin receptor 3",
  "term_id": "GO:0005737",
  "gene": "UniProtKB:P41968",
  "gene_symbol": "MC3R"
}